{
  "gene": "UniProtKB:Q9ULR5",
  "term_id": "GO:0017148",
  "term_label": "negative regulation of translation",
  "gene_symbol": "PAIP2B",
  "gene_name": "Polyadenylate-binding protein-interacting protein 2B"
}